myeloid leukocyte mediated immunity [GO:0002444] (biological process) Sources: GOC:add, GO_REF:0000022, ISBN:0781735149 Definition: Any process involved in the carrying out of an immune response by a myeloid leukocyte. Relationships: is a type of GO:0002443 Also known as: myeloid leucocyte immune effector process, myeloid leucocyte mediated immunity, myeloid leukocyte immune effector process Subtypes: type III hypersensitivity [GO:0001802], myeloid dendritic cell cytokine production [GO:0002372], type II hypersensitivity [GO:0002445], neutrophil mediated immunity [GO:0002446], eosinophil mediated immunity [GO:0002447], mast cell mediated immunity [GO:0002448], basophil mediated immunity [GO:0002560], microglial cell mediated cytotoxicity [GO:0090634] Regulation: regulated by regulation of myeloid leukocyte mediated immunity [GO:0002886]; negatively regulated by negative regulation of myeloid leukocyte mediated immunity [GO:0002887]; positively regulated by positive regulation of myeloid leukocyte mediated immunity [GO:0002888]